{
  "term_label": "structural constituent of ribosome",
  "gene_symbol": "MRPL20",
  "gene": "UniProtKB:Q9BYC9",
  "gene_name": "Large ribosomal subunit protein bL20m",
  "term_id": "GO:0003735"
}